DNA replication origin binding [GO:0003688] (molecular function) Relationships: is a type of sequence-specific double-stranded DNA binding [GO:1990837] Definition: Binding to a DNA replication origin, a unique DNA sequence of a replicon at which DNA replication is initiated and proceeds bidirectionally or unidirectionally. Also known as: ARS binding Sources: GOC:curators